{
  "gene_name": "Succinate--CoA ligase [ADP_GDP-forming] subunit alpha, mitochondrial",
  "term_label": "succinate-CoA ligase (GDP-forming) activity",
  "gene": "UniProtKB:P53597",
  "gene_symbol": "SUCLG1",
  "term_id": "GO:0004776"
}